D-amino-acid dehydrogenase activity [GO:0008718] (molecular function) Also known as: D-amino-acid:(acceptor) oxidoreductase (deaminating), D-amino-acid:acceptor oxidoreductase (deaminating) Relationships: is a type of oxidoreductase activity, acting on the CH-NH2 group of donors [GO:0016638] Sources: RHEA:18125 Definition: Catalysis of the reaction: a D-amino acid + H2O + acceptor = a 2-oxo acid + NH3 + reduced acceptor.